(E,E)-geranyllinalool synthase activity [GO:0080013] (molecular function) Definition: Catalysis of the reaction: all-trans-geranyl-geranyl diphosphate + H2O = (E,E)-geranyllinalool + diphosphate. References: PMID:18398052 Sources: MetaCyc:RXN-10441 Relationships: is a type of carbon-oxygen lyase activity, acting on phosphates [GO:0016838]